{
  "gene_name": "Syntaxin-binding protein 5",
  "term_label": "plasma membrane",
  "gene": "UniProtKB:Q5T5C0",
  "term_id": "GO:0005886",
  "gene_symbol": "STXBP5"
}